regulatory ncRNA 3'-end processing [GO:0043628] (biological process) Definition: Any process involved in forming the mature 3' end of a regulatory non-coding RNA molecule. Subtypes: pre-miRNA 3'-end processing [GO:0044747], GO:1990431, siRNA 3'-end processing [GO:1990432] Sources: GOC:jl Also known as: ncRNA 3' end processing, ncRNA 3'-end processing, small regulatory ncRNA 3'-end processing Relationships: is a type of GO:0031123; is a type of regulatory ncRNA processing [GO:0070918]